{
  "gene_name": "Guanine nucleotide exchange factor for Rab-3A",
  "term_id": "UNKNOWN:0002",
  "gene": "UniProtKB:Q8TBN0",
  "gene_symbol": "RAB3IL1",
  "term_label": "Unknown biological process"
}